{
  "gene": "UniProtKB:Q8N5H3",
  "term_label": "negative regulation of transforming growth factor beta receptor signaling pathway",
  "gene_name": "Leucine repeat adapter protein 25",
  "term_id": "GO:0030512",
  "gene_symbol": "FAM89B"
}